{
  "term_id": "GO:0010494",
  "gene_symbol": "FMR1",
  "gene_name": "Fragile X messenger ribonucleoprotein 1",
  "term_label": "cytoplasmic stress granule",
  "gene": "UniProtKB:Q06787"
}